mating-type factor pheromone receptor activity [GO:0004932] (molecular function) Sources: GOC:dph, GOC:vw Subtypes: mating-type a-factor pheromone receptor activity [GO:0004933], mating-type alpha-factor pheromone receptor activity [GO:0004934], mating-type M-factor pheromone receptor activity [GO:0036319], mating-type P-factor pheromone receptor activity [GO:0036320] Definition: Combining with a mating-type factor pheromone to initiate a change in cell activity. Relationships: is a type of G protein-coupled peptide receptor activity [GO:0008528]; is a type of pheromone receptor activity [GO:0016503]